{
  "gene_symbol": "ATP9B",
  "gene_name": "Probable phospholipid-transporting ATPase IIB",
  "term_label": "trans-Golgi network",
  "term_id": "GO:0005802",
  "gene": "UniProtKB:O43861"
}